{
  "gene_name": "Nuclear receptor subfamily 2 group C member 2",
  "term_id": "GO:0000978",
  "gene": "UniProtKB:P49116",
  "term_label": "RNA polymerase II cis-regulatory region sequence-specific DNA binding",
  "gene_symbol": "NR2C2"
}